{
  "term_id": "GO:0000981",
  "gene_symbol": "IRF3",
  "term_label": "DNA-binding transcription factor activity, RNA polymerase II-specific",
  "gene_name": "Interferon regulatory factor 3",
  "gene": "UniProtKB:Q14653"
}